{
  "gene_name": "Kinocilin",
  "term_id": "GO:0032437",
  "term_label": "cuticular plate",
  "gene": "UniProtKB:A6PVL3",
  "gene_symbol": "KNCN"
}